venom-mediated inhibition of voltage-gated calcium channel activity [GO:0044474] (biological process) Also known as: envenomation resulting in negative regulation of voltage-gated calcium channel activity in another organism, envenomation resulting in negative regulation of voltage-gated calcium channel activity in other organism References: PMID:20920515 Sources: GOC:fj, GOC:jl Subtypes: venom-mediated inhibition of high voltage-gated calcium channel activity [GO:0044475], GO:0044476 Relationships: is a type of venom-mediated inhibition of calcium channel activity [GO:0044473] Definition: A process in which an organism inhibits or disrupts the activity of a voltage-gated calcium channel in another organism via the action of a venom.